{
  "term_id": "GO:0005654",
  "gene_name": "EP300-interacting inhibitor of differentiation 2",
  "gene": "UniProtKB:Q8N6I1",
  "gene_symbol": "EID2",
  "term_label": "nucleoplasm"
}